{
  "gene_name": "Calcineurin subunit B type 1",
  "term_id": "GO:0005955",
  "gene_symbol": "PPP3R1",
  "term_label": "calcineurin complex",
  "gene": "UniProtKB:P63098"
}